{
  "gene": "UniProtKB:Q8IY31",
  "term_label": "cytoplasm",
  "gene_symbol": "IFT20",
  "gene_name": "Intraflagellar transport protein 20 homolog",
  "term_id": "GO:0005737"
}